{
  "term_label": "cytokine activity",
  "gene": "UniProtKB:Q92838",
  "term_id": "GO:0005125",
  "gene_name": "Ectodysplasin-A",
  "gene_symbol": "EDA"
}